short-chain fatty acid transmembrane transporter activity [GO:0015636] (molecular function) Relationships: is a type of fatty acid transmembrane transporter activity [GO:0015245]; is part of short-chain fatty acid transport [GO:0015912] Definition: Enables the transfer of short-chain fatty acids from one side of a membrane to the other. A short-chain fatty acid has an aliphatic tail containing fewer than 6 carbons. Sources: GOC:mah Note: While there is not universal consensus on the lengths of short-, medium-, long- and very-long-chain fatty acids, the GO uses the definitions in ChEBI (see CHEBI:26666, CHEBI:59554, CHEBI:15904 and CHEBI:27283). Also known as: short-chain fatty acid transporter activity, short-chain fatty acid uptake transporter activity Subtypes: propionate transmembrane transporter activity [GO:0015552]